{
  "gene": "UniProtKB:Q06481",
  "term_label": "Unknown cellular component",
  "term_id": "UNKNOWN:0003",
  "gene_symbol": "APLP2",
  "gene_name": "Amyloid beta precursor like protein 2"
}